{
  "gene_symbol": "CNBD2",
  "term_id": "GO:0030552",
  "gene_name": "Cyclic nucleotide-binding domain-containing protein 2",
  "term_label": "cAMP binding",
  "gene": "UniProtKB:Q96M20"
}